{
  "term_id": "GO:0004888",
  "gene": "UniProtKB:Q9H7L2",
  "gene_name": "Putative killer cell immunoglobulin-like receptor-like protein KIR3DX1",
  "gene_symbol": "KIR3DX1",
  "term_label": "transmembrane signaling receptor activity"
}